{
  "gene_symbol": "GH2",
  "gene": "UniProtKB:P01242",
  "term_label": "extracellular space",
  "term_id": "GO:0005615",
  "gene_name": "Growth hormone variant"
}